{
  "term_label": "anaphase-promoting complex",
  "gene_name": "Anaphase-promoting complex subunit 1",
  "term_id": "GO:0005680",
  "gene": "UniProtKB:Q9H1A4",
  "gene_symbol": "ANAPC1"
}